{
  "term_id": "GO:0008474",
  "term_label": "palmitoyl-(protein) hydrolase activity",
  "gene": "UniProtKB:Q6PCB6",
  "gene_symbol": "ABHD17C",
  "gene_name": "Alpha_beta hydrolase domain-containing protein 17C"
}